{
  "gene": "UniProtKB:Q14596",
  "term_id": "GO:0016236",
  "gene_name": "Next to BRCA1 gene 1 protein",
  "gene_symbol": "NBR1",
  "term_label": "macroautophagy"
}